{
  "gene_symbol": "NLRP11",
  "term_label": "Unknown molecular function",
  "gene_name": "NACHT, LRR and PYD domains-containing protein 11",
  "term_id": "UNKNOWN:0001",
  "gene": "UniProtKB:P59045"
}